positive regulation of thiamine biosynthetic process [GO:0090180] (biological process) Sources: GOC:dph, GOC:tb Definition: Any process that increases the frequency, rate or extent of the chemical reactions and pathways resulting in the formation of thiamine. Relationships: is a type of positive regulation of vitamin metabolic process [GO:0046136]; is a type of GO:0070623; is a type of positive regulation of alcohol biosynthetic process [GO:1902932]; RO_0002213 thiamine biosynthetic process [GO:0009228] Also known as: positive regulation of thiamin biosynthetic process